{
  "term_label": "eosinophil chemotaxis",
  "term_id": "GO:0048245",
  "gene_name": "Eotaxin",
  "gene": "UniProtKB:P51671",
  "gene_symbol": "CCL11"
}